oscillatory muscle contraction [GO:0014703] (biological process) Sources: GOC:mtg_muscle Definition: A process in which force is generated within oscillatory skeletal muscle tissue, resulting in a change in muscle geometry. Force generation involves a chemo-mechanical energy conversion step that is carried out by the actin/myosin complex activity, which generates force through ATP hydrolysis. Oscillatory muscle contraction occurs in insect wing muscles and is characterized by asynchrony between action potential and contraction and by stretch activation. Relationships: is a type of voluntary skeletal muscle contraction [GO:0003010]